cellular response to sorbitol [GO:0072709] (biological process) Definition: Any process that results in a change in state or activity of a cell (in terms of movement, secretion, enzyme production, gene expression, etc.) as a result of a sorbitol stimulus. Sources: GOC:mah Relationships: is a type of cellular response to carbohydrate stimulus [GO:0071322]; is a type of response to sorbitol [GO:0072708] Also known as: cellular response to glucitol